positive regulation of protein neddylation [GO:2000436] (biological process) Sources: GOC:obol Also known as: positive regulation of RUB1-protein conjugation Definition: Any process that activates or increases the frequency, rate or extent of protein neddylation. Relationships: is a type of positive regulation of protein modification by small protein conjugation or removal [GO:1903322]; is a type of regulation of protein neddylation [GO:2000434]; positively regulates protein neddylation [GO:0045116]